{
  "gene_symbol": "PIGU",
  "gene": "UniProtKB:Q9H490",
  "gene_name": "Phosphatidylinositol glycan anchor biosynthesis class U protein",
  "term_id": "GO:0016255",
  "term_label": "attachment of GPI anchor to protein"
}